host cell presynaptic membrane [GO:0044231] (cellular component) Sources: GOC:rph Also known as: host cell pre-synaptic membrane, other organism pre-synaptic membrane, other organism presynaptic membrane Definition: A specialized area of membrane of the host axon terminal that faces the plasma membrane of the host neuron or muscle fiber with which the axon terminal establishes a synaptic junction; many host synaptic junctions exhibit structural presynaptic characteristics, such as conical, electron-dense internal protrusions, that distinguish it from the remainder of the axon plasma membrane. Relationships: is a type of host cell part [GO:0033643]; is part of host cell membrane [GO:0033644]; is part of host cell synapse [GO:0044221]